{
  "term_label": "Unknown cellular component",
  "term_id": "UNKNOWN:0003",
  "gene": "UniProtKB:Q15165",
  "gene_name": "Serum paraoxonase_arylesterase 2",
  "gene_symbol": "PON2"
}